{
  "gene_name": "Achaete-scute homolog 4",
  "gene_symbol": "ASCL4",
  "gene": "UniProtKB:Q6XD76",
  "term_label": "regulation of transcription by RNA polymerase II",
  "term_id": "GO:0006357"
}